{
  "gene_name": "SH3 and cysteine-rich domain-containing protein",
  "gene": "UniProtKB:Q99469",
  "gene_symbol": "STAC",
  "term_label": "positive regulation of protein localization to plasma membrane",
  "term_id": "GO:1903078"
}